{
  "gene_name": "LIM and calponin homology domains-containing protein 1",
  "term_label": "positive regulation of stress fiber assembly",
  "gene": "UniProtKB:Q9UPQ0",
  "gene_symbol": "LIMCH1",
  "term_id": "GO:0051496"
}